{
  "gene_symbol": "FLAD1",
  "gene": "UniProtKB:Q8NFF5",
  "term_label": "Unknown cellular component",
  "gene_name": "FAD synthase",
  "term_id": "UNKNOWN:0003"
}